{
  "gene": "UniProtKB:P78424",
  "gene_name": "POU domain, class 6, transcription factor 2",
  "gene_symbol": "POU6F2",
  "term_id": "UNKNOWN:0003",
  "term_label": "Unknown cellular component"
}